{
  "gene": "UniProtKB:Q9NVV2",
  "gene_symbol": "C19orf73",
  "term_id": "UNKNOWN:0003",
  "term_label": "Unknown cellular component",
  "gene_name": "Putative uncharacterized protein C19orf73"
}